{
  "gene_symbol": "PPY",
  "term_id": "GO:0007631",
  "gene_name": "Pancreatic polypeptide prohormone",
  "gene": "UniProtKB:P01298",
  "term_label": "feeding behavior"
}